nickel cation import across plasma membrane [GO:0098716] (biological process) Also known as: nickel cation import into cell Definition: The directed movement of nickel cations from outside of a cell, across the plasma membrane and into the cytosol. Relationships: is a type of GO:0035444; is a type of GO:0098659 Sources: GOC:dos